{
  "gene": "UniProtKB:Q9UBN1",
  "gene_symbol": "CACNG4",
  "term_id": "GO:0098839",
  "term_label": "postsynaptic density membrane",
  "gene_name": "Voltage-dependent calcium channel gamma-4 subunit"
}